type 4 metabotropic glutamate receptor binding [GO:0031801] (molecular function) Sources: GOC:mah, GOC:nln Relationships: is a type of G protein-coupled glutamate receptor binding [GO:0035256] Definition: Binding to a type 4 metabotropic glutamate receptor. Also known as: type 4 metabotropic glutamate receptor ligand